{
  "gene_symbol": "SLC26A2",
  "term_label": "chloride transmembrane transport",
  "gene": "UniProtKB:P50443",
  "term_id": "GO:1902476",
  "gene_name": "Sulfate transporter"
}